{
  "term_label": "neuromuscular junction",
  "term_id": "GO:0031594",
  "gene_name": "Disks large homolog 2",
  "gene": "UniProtKB:Q15700",
  "gene_symbol": "DLG2"
}